{
  "term_id": "UNKNOWN:0001",
  "gene_symbol": "VWA5B2",
  "term_label": "Unknown molecular function",
  "gene_name": "von Willebrand factor A domain-containing protein 5B2",
  "gene": "UniProtKB:Q8N398"
}